{
  "term_label": "protein N-linked glycosylation",
  "gene": "UniProtKB:Q5I7T1",
  "gene_name": "Putative Dol-P-Glc:Glc(2)Man(9)GlcNAc(2)-PP-Dol alpha-1,2-glucosyltransferase",
  "gene_symbol": "ALG10B",
  "term_id": "GO:0006487"
}